{
  "gene_symbol": "BCLAF1",
  "term_id": "GO:0045944",
  "term_label": "positive regulation of transcription by RNA polymerase II",
  "gene": "UniProtKB:Q9NYF8",
  "gene_name": "Bcl-2-associated transcription factor 1"
}